negative regulation of peripheral T cell tolerance induction [GO:0002850] (biological process) Subtypes: GO:0002847 Also known as: down regulation of peripheral T cell tolerance induction, down-regulation of peripheral T cell tolerance induction, downregulation of peripheral T cell tolerance induction, inhibition of peripheral T cell tolerance induction Definition: Any process that stops, prevents, or reduces the frequency, rate, or extent of peripheral T cell tolerance induction. Sources: GOC:add Relationships: is a type of negative regulation of peripheral tolerance induction [GO:0002659]; is a type of negative regulation of T cell tolerance induction [GO:0002665]; is_a negative regulation of T cell mediated immunity [GO:0002710]; is a type of regulation of peripheral T cell tolerance induction [GO:0002849]; negatively regulates GO:0002458